{
  "gene": "UniProtKB:Q15485",
  "term_label": "antigen binding",
  "gene_symbol": "FCN2",
  "gene_name": "Ficolin-2",
  "term_id": "GO:0003823"
}